{
  "term_id": "GO:0043153",
  "gene": "UniProtKB:Q9UKT7",
  "gene_symbol": "FBXL3",
  "term_label": "entrainment of circadian clock by photoperiod",
  "gene_name": "F-box_LRR-repeat protein 3"
}